beta-1,3-galactosyltransferase activity [GO:0048531] (molecular function) References: PMID:11551958 Relationships: is a type of galactosyltransferase activity [GO:0008378] Subtypes: N-acetyl-beta-D-glucosaminide beta-(1,3)-galactosyltransferase activity [GO:0008499], glycoprotein-N-acetylgalactosamine 3-beta-galactosyltransferase activity [GO:0016263], GO:0047240 Definition: Catalysis of the transfer of a galactose residue from a donor molecule to an oligosaccharide, forming a beta-1,3-linkage.